{
  "gene_name": "Axonemal dynein light intermediate polypeptide 1",
  "term_label": "ciliary base",
  "term_id": "GO:0097546",
  "gene": "UniProtKB:O14645",
  "gene_symbol": "DNALI1"
}